{
  "gene_name": "Tumor necrosis factor receptor superfamily member 1A",
  "term_label": "tumor necrosis factor binding",
  "gene": "UniProtKB:P19438",
  "term_id": "GO:0043120",
  "gene_symbol": "TNFRSF1A"
}